{
  "gene": "UniProtKB:Q9H900",
  "gene_name": "Protein zwilch homolog",
  "gene_symbol": "ZWILCH",
  "term_id": "UNKNOWN:0001",
  "term_label": "Unknown molecular function"
}